cation channel complex [GO:0034703] (CC) Sources: GOC:mah Definition: An ion channel complex through which cations pass. Relationships: is a type of monoatomic ion channel complex [GO:0034702] Subtypes: intracellular cyclic nucleotide activated cation channel complex [GO:0017071], calcium channel complex [GO:0034704], GO:0034705, sodium channel complex [GO:0034706], proton-transporting ATP synthase complex [GO:0045259], GO:1904602